{
  "term_label": "Unknown molecular function",
  "gene_name": "Negative elongation factor E",
  "gene_symbol": "NELFE",
  "term_id": "UNKNOWN:0001",
  "gene": "UniProtKB:P18615"
}